{
  "term_id": "UNKNOWN:0001",
  "gene": "UniProtKB:Q8NFU4",
  "term_label": "Unknown molecular function",
  "gene_name": "Follicular dendritic cell secreted peptide",
  "gene_symbol": "FDCSP"
}